{
  "gene_symbol": "ID3",
  "gene_name": "DNA-binding protein inhibitor ID-3",
  "term_id": "GO:0005634",
  "term_label": "nucleus",
  "gene": "UniProtKB:Q02535"
}